{
  "term_id": "UNKNOWN:0001",
  "gene": "UniProtKB:Q6PIY5",
  "term_label": "Unknown molecular function",
  "gene_symbol": "ARMH1",
  "gene_name": "Armadillo-like helical domain containing protein 1"
}